rhabdomere membrane [GO:0033583] (cellular component) Definition: The portion of the plasma membrane surrounding the rhabdomere. Sources: GOC:mah Relationships: is a type of cell projection membrane [GO:0031253]; is part of GO:0016028